extrinsic component of external side of plasma membrane [GO:0031232] (cellular component) Also known as: extrinsic to external leaflet of plasma membrane, extrinsic to external side of plasma membrane Subtypes: extrinsic component of periplasmic side of plasma membrane [GO:0031236] Definition: The component of a plasma membrane consisting of gene products and protein complexes that are loosely bound to its external surface, but not integrated into the hydrophobic region. Relationships: is a type of extrinsic component of plasma membrane [GO:0019897]; is part of external side of plasma membrane [GO:0009897] Sources: GOC:dos, GOC:mah